{
  "gene_symbol": "ACTL8",
  "term_id": "GO:0015629",
  "gene_name": "Actin-like protein 8",
  "gene": "UniProtKB:Q9H568",
  "term_label": "actin cytoskeleton"
}